{
  "gene": "UniProtKB:Q969P5",
  "term_id": "GO:0005634",
  "term_label": "nucleus",
  "gene_symbol": "FBXO32",
  "gene_name": "F-box only protein 32"
}